propionyl-CoA:succinate CoA-transferase activity [GO:0043821] (molecular function) Relationships: is a type of GO:0008410 Also known as: propionyl-CoA succinate CoA-transferase activity, propionyl-CoA:succinate CoA transferase activity Definition: Catalysis of the reaction: succinate + propionyl-CoA = succinyl-CoA + propionate. References: PMID:10769117